{
  "term_label": "nucleoplasm",
  "gene_name": "Metastasis-associated protein MTA1",
  "gene": "UniProtKB:Q13330",
  "term_id": "GO:0005654",
  "gene_symbol": "MTA1"
}